{
  "gene": "UniProtKB:Q07092",
  "gene_name": "Collagen alpha-1(XVI) chain",
  "term_id": "GO:0005604",
  "term_label": "basement membrane",
  "gene_symbol": "COL16A1"
}